{
  "gene": "UniProtKB:Q9NRE2",
  "gene_symbol": "TSHZ2",
  "gene_name": "Teashirt homolog 2",
  "term_id": "GO:0003677",
  "term_label": "DNA binding"
}